{
  "gene": "UniProtKB:Q8N4B4",
  "term_id": "GO:0031146",
  "term_label": "SCF-dependent proteasomal ubiquitin-dependent protein catabolic process",
  "gene_name": "F-box only protein 39",
  "gene_symbol": "FBXO39"
}